{
  "term_label": "cytoplasm",
  "gene_name": "G-protein coupled receptor 6",
  "gene": "UniProtKB:P46095",
  "term_id": "GO:0005737",
  "gene_symbol": "GPR6"
}